{
  "term_id": "GO:0016192",
  "gene_name": "C-Jun-amino-terminal kinase-interacting protein 3",
  "term_label": "vesicle-mediated transport",
  "gene": "UniProtKB:Q9UPT6",
  "gene_symbol": "MAPK8IP3"
}